{
  "gene_symbol": "FUBP1",
  "term_label": "mRNA 3'-UTR binding",
  "gene_name": "Far upstream element-binding protein 1",
  "gene": "UniProtKB:Q96AE4",
  "term_id": "GO:0003730"
}